serine import across plasma membrane [GO:0098718] (biological process) Also known as: serine import into cell Sources: GOC:dos Definition: The directed movement of serine from outside of a cell, across the plasma membrane and into the cytosol. Subtypes: L-serine import across plasma membrane [GO:1903812] Relationships: is a type of GO:0032329; is a type of amino acid import across plasma membrane [GO:0089718]; is a type of carboxylic acid transmembrane transport [GO:1905039]